{
  "gene": "UniProtKB:O75925",
  "gene_name": "E3 SUMO-protein ligase PIAS1",
  "gene_symbol": "PIAS1",
  "term_label": "transcription coregulator activity",
  "term_id": "GO:0003712"
}